{
  "gene_symbol": "MARS1",
  "gene_name": "Methionine--tRNA ligase, cytoplasmic",
  "term_label": "methionine-tRNA ligase activity",
  "gene": "UniProtKB:P56192",
  "term_id": "GO:0004825"
}